{
  "term_id": "GO:0015711",
  "term_label": "organic anion transport",
  "gene": "UniProtKB:Q5T3U5",
  "gene_symbol": "ABCC10",
  "gene_name": "ATP-binding cassette sub-family C member 10"
}